{
  "gene_name": "Phosphatidate phosphatase LPIN1",
  "gene": "UniProtKB:Q14693",
  "gene_symbol": "LPIN1",
  "term_label": "nucleus",
  "term_id": "GO:0005634"
}